{
  "gene_name": "Zinc finger protein 594",
  "term_label": "nucleus",
  "gene_symbol": "ZNF594",
  "gene": "UniProtKB:Q96JF6",
  "term_id": "GO:0005634"
}